{
  "term_id": "GO:0141156",
  "gene": "UniProtKB:Q03060",
  "gene_name": "cAMP-responsive element modulator",
  "term_label": "cAMP/PKA signal transduction",
  "gene_symbol": "CREM"
}